purine nucleoside binding [GO:0001883] (molecular function) Subtypes: purine deoxyribonucleoside binding [GO:0032547], purine ribonucleoside binding [GO:0032550] Definition: Binding to a purine nucleoside, a compound consisting of a purine base linked either to ribose or deoxyribose. Sources: GOC:hjd Relationships: is a type of nucleoside binding [GO:0001882]